{
  "gene_name": "Zinc finger protein ZFP2",
  "gene_symbol": "ZFP2",
  "term_label": "DNA-binding transcription factor activity, RNA polymerase II-specific",
  "term_id": "GO:0000981",
  "gene": "UniProtKB:Q6ZN57"
}